{
  "gene": "UniProtKB:Q5T6R2",
  "term_id": "UNKNOWN:0003",
  "gene_symbol": "TPTE2P1",
  "term_label": "Unknown cellular component",
  "gene_name": "Putative phosphatidylinositol 3,4,5-trisphosphate 3-phosphatase TPTE2P1"
}